{
  "term_label": "Unknown biological process",
  "gene": "UniProtKB:Q9NSP4",
  "gene_name": "Centromere protein M",
  "gene_symbol": "CENPM",
  "term_id": "UNKNOWN:0002"
}